{
  "gene_name": "RNA-binding protein RO60",
  "gene": "UniProtKB:P10155",
  "gene_symbol": "RO60",
  "term_id": "GO:1990904",
  "term_label": "ribonucleoprotein complex"
}